{
  "term_label": "amyloid-beta binding",
  "gene_symbol": "ITM2A",
  "gene": "UniProtKB:O43736",
  "term_id": "GO:0001540",
  "gene_name": "Integral membrane protein 2A"
}